{
  "term_id": "GO:1902237",
  "term_label": "positive regulation of endoplasmic reticulum stress-induced intrinsic apoptotic signaling pathway",
  "gene_symbol": "NCK1",
  "gene_name": "Cytoplasmic protein NCK1",
  "gene": "UniProtKB:P16333"
}